{
  "gene": "UniProtKB:Q96AC6",
  "gene_name": "Kinesin-like protein KIFC2",
  "gene_symbol": "KIFC2",
  "term_label": "kinesin complex",
  "term_id": "GO:0005871"
}